{
  "gene_name": "Putative DBH-like monooxygenase protein 2",
  "gene_symbol": "MOXD2P",
  "gene": "UniProtKB:A6NHM9",
  "term_id": "GO:0042421",
  "term_label": "norepinephrine biosynthetic process"
}